cerebellar Golgi cell differentiation [GO:0021701] (biological process) References: PMID:15157725 Sources: GOC:cls, GOC:dgh, GOC:dph, GOC:jid, GO_REF:0000021 Definition: The process in which neuroblasts acquire specialized structural and/or functional features that characterize the mature cerebellar Golgi cell. Differentiation includes the processes involved in commitment of a neuroblast to a Golgi cell fate. A cerebellar Golgi cell is an inhibitory GABAergic interneuron found in the cerebellar cortex. Relationships: is a type of cell differentiation in hindbrain [GO:0021533]; is a type of central nervous system neuron differentiation [GO:0021953]; is a type of GABAergic neuron differentiation [GO:0097154]; BFO_0000050 cerebellar granular layer formation [GO:0021684]